negative regulation of muscle organ development [GO:0048635] (biological process) Also known as: down regulation of muscle development, down-regulation of muscle development, downregulation of muscle development, inhibition of muscle development Sources: GOC:go_curators Relationships: is a type of regulation of muscle organ development [GO:0048634]; is a type of GO:0051093; is a type of negative regulation of multicellular organismal process [GO:0051241]; negatively regulates muscle organ development [GO:0007517] Subtypes: negative regulation of somitomeric trunk muscle development [GO:0014710], negative regulation of striated muscle tissue development [GO:0045843] Definition: Any process that stops, prevents, or reduces the frequency, rate or extent of muscle development.